{
  "gene_symbol": "SLC14A2",
  "term_label": "Unknown cellular component",
  "gene_name": "Urea transporter 2",
  "gene": "UniProtKB:Q15849",
  "term_id": "UNKNOWN:0003"
}